{
  "gene_name": "Olfactory receptor 2S2",
  "term_label": "olfactory receptor activity",
  "gene": "UniProtKB:Q9NQN1",
  "gene_symbol": "OR2S2",
  "term_id": "GO:0004984"
}